GDP-dissociation inhibitor binding [GO:0051021] (molecular function) Definition: Binding to a GDP-dissociation inhibitor protein. Sources: GOC:ai Subtypes: Rho GDP-dissociation inhibitor binding [GO:0051022] Also known as: GDI binding Relationships: is a type of GO:0005515